{
  "term_label": "Unknown molecular function",
  "gene_symbol": "HAUS1",
  "gene": "UniProtKB:Q96CS2",
  "gene_name": "HAUS augmin-like complex subunit 1",
  "term_id": "UNKNOWN:0001"
}